{
  "gene_symbol": "MRPL27",
  "term_id": "UNKNOWN:0002",
  "gene": "UniProtKB:Q9P0M9",
  "term_label": "Unknown biological process",
  "gene_name": "Large ribosomal subunit protein bL27m"
}